P-type proton-exporting transporter activity [GO:0008553] (MF) Subtypes: P-type potassium:proton transporter activity [GO:0008900] Also known as: H+-transporting ATPase, H+-transporting ATPase activity, P-type H+-exporting ATPase activity, hydrogen-exporting ATPase activity, proton-exporting ATPase activity, hydrogen exporting ATPase activity, phosphorylative mechanism, proton-transporting ATPase activity, H+-exporting ATPase activity, hydrogen-/sodium-translocating ATPase activity, hydrogen-exporting ATPase activity, phosphorylative mechanism, proton transport ATPase activity, proton-exporting ATPase activity, phosphorylative mechanism, proton-translocating ATPase activity Sources: RHEA:20852 Relationships: is a type of proton transmembrane transporter activity [GO:0015078]; is_a P-type ion transporter activity [GO:0015662]; is a type of GO:0019829 Definition: Enables the transfer of protons from one side of a membrane to the other according to the reaction: ATP + H2O + H+(in) = ADP + phosphate + H+(out). These transporters use a phosphorylative mechanism, which have a phosphorylated intermediate state during the ion transport cycle.